Golgi vesicle budding [GO:0048194] (biological process) Relationships: is a type of vesicle budding from membrane [GO:0006900]; is part of Golgi vesicle transport [GO:0048193]; occurs in Golgi membrane [GO:0000139] Also known as: Golgi-derived vesicle budding, dictyosome vesicle budding Definition: The evagination of the Golgi membrane, resulting in formation of a vesicle. References: PMID:10219233 Sources: GOC:jid, ISBN:0716731363